{
  "term_label": "DNA-binding transcription factor activity, RNA polymerase II-specific",
  "gene": "UniProtKB:P10243",
  "gene_name": "Myb-related protein A",
  "term_id": "GO:0000981",
  "gene_symbol": "MYBL1"
}